{
  "gene_symbol": "SLC6A9",
  "term_label": "amino acid:sodium symporter activity",
  "gene_name": "Sodium- and chloride-dependent glycine transporter 1",
  "gene": "UniProtKB:P48067",
  "term_id": "GO:0005283"
}